{
  "gene_symbol": "RPS20",
  "term_id": "GO:0003735",
  "term_label": "structural constituent of ribosome",
  "gene_name": "Small ribosomal subunit protein uS10",
  "gene": "UniProtKB:P60866"
}